{
  "gene": "UniProtKB:Q9Y576",
  "term_label": "ubiquitin ligase complex",
  "gene_symbol": "ASB1",
  "term_id": "GO:0000151",
  "gene_name": "Ankyrin repeat and SOCS box protein 1"
}